{
  "gene": "UniProtKB:O14503",
  "term_id": "GO:0000122",
  "gene_symbol": "BHLHE40",
  "term_label": "negative regulation of transcription by RNA polymerase II",
  "gene_name": "Class E basic helix-loop-helix protein 40"
}